cardiac cell fate determination [GO:0060913] (biological process) Definition: The process involved in cardiac cell fate commitment. Once determination has taken place, a cell becomes committed to differentiate down a particular pathway regardless of its environment. Sources: GOC:mtg_heart Also known as: cardiocyte cell fate determination Subtypes: cardioblast cell fate determination [GO:0007510], cardiac muscle cell fate determination [GO:0061442], endocardial cushion cell fate determination [GO:0061446] Relationships: is a type of cell fate determination [GO:0001709]; is part of GO:0060911